{
  "gene_symbol": "NLRP1",
  "gene": "UniProtKB:Q9C000",
  "gene_name": "NACHT, LRR and PYD domains-containing protein 1",
  "term_label": "pattern recognition receptor activity",
  "term_id": "GO:0038187"
}